positive regulation of cardiac muscle adaptation [GO:0010615] (biological process) Definition: Any process that increases the rate, extent or frequency of the process in which cardiac muscle adapts, with consequent modifications to structural and/or functional phenotypes, in response to a stimulus. Stimuli include contractile activity, loading conditions, substrate supply, and environmental factors. Sources: GOC:BHF, GOC:dph, GOC:tb Relationships: is a type of regulation of cardiac muscle adaptation [GO:0010612]; is a type of positive regulation of muscle adaptation [GO:0014744]; positively regulates cardiac muscle adaptation [GO:0014887] Subtypes: positive regulation of cardiac muscle hypertrophy in response to stress [GO:1903244]